mannosylglycerate hydrolase activity [GO:0102546] (molecular function) Relationships: is a type of GO:0016803 Sources: RHEA:58456 Definition: Catalysis of the reaction: (2R)-2-O-(alpha-D-mannosyl)-glycerate + H2O = (R)-glycerate + D-mannose.